{
  "gene_name": "T cell receptor delta joining 3 (Fragment)",
  "gene": "UniProtKB:A0A075B6W1",
  "term_id": "UNKNOWN:0001",
  "gene_symbol": "TRDJ3",
  "term_label": "Unknown molecular function"
}